{
  "term_label": "Unknown cellular component",
  "gene_symbol": "CFAP68",
  "gene": "UniProtKB:Q9H5F2",
  "term_id": "UNKNOWN:0003",
  "gene_name": "Cilia- and flagella-associated protein 68"
}